{
  "gene_name": "Ubiquitin carboxyl-terminal hydrolase 4",
  "term_label": "nucleus",
  "gene_symbol": "USP4",
  "term_id": "GO:0005634",
  "gene": "UniProtKB:Q13107"
}